{
  "gene": "UniProtKB:Q9NQS7",
  "gene_name": "Inner centromere protein",
  "term_id": "GO:0000776",
  "gene_symbol": "INCENP",
  "term_label": "kinetochore"
}